negative regulation of response to benzene [GO:1901452] (biological process) Relationships: is a type of negative regulation of response to stimulus [GO:0048585]; is a type of GO:1901451; negatively regulates GO:1901423 Definition: Any process that stops, prevents or reduces the frequency, rate or extent of response to benzene. Sources: GOC:TermGenie, GOC:mengo_curators Also known as: down regulation of response to benzene, down-regulation of response to benzene, downregulation of response to benzene, inhibition of response to benzene